{
  "gene_symbol": "BTBD7",
  "term_label": "regulation of branching involved in salivary gland morphogenesis",
  "term_id": "GO:0060693",
  "gene": "UniProtKB:Q9P203",
  "gene_name": "BTB_POZ domain-containing protein 7"
}